{
  "term_label": "Unknown molecular function",
  "gene_name": "NADH dehydrogenase [ubiquinone] 1 alpha subcomplex assembly factor 2",
  "gene": "UniProtKB:Q8N183",
  "gene_symbol": "NDUFAF2",
  "term_id": "UNKNOWN:0001"
}